{
  "gene_symbol": "OR4A5",
  "gene": "UniProtKB:Q8NH83",
  "term_id": "GO:0005886",
  "term_label": "plasma membrane",
  "gene_name": "Olfactory receptor 4A5"
}